{
  "term_label": "cytoplasm",
  "term_id": "GO:0005737",
  "gene_symbol": "GSTCD",
  "gene_name": "Glutathione S-transferase C-terminal domain-containing protein",
  "gene": "UniProtKB:Q8NEC7"
}